helper T cell enhancement of B cell mediated immune response [GO:0035399] (biological process) Definition: Positive regulation of a B cell mediated immune response mediated via cytokine production by a helper T cell. Sources: GOC:add Relationships: is a type of positive regulation of B cell mediated immunity [GO:0002714]; is a type of helper T cell enhancement of adaptive immune response [GO:0035397] Also known as: helper T cell enhancement of B cell mediated immunity, provision of T cell help to B cell